{
  "gene": "UniProtKB:P04432",
  "gene_symbol": "IGKV1D-39",
  "term_id": "GO:0019814",
  "term_label": "immunoglobulin complex",
  "gene_name": "Immunoglobulin kappa variable 1D-39"
}